{
  "term_label": "adenylate cyclase-activating adrenergic receptor signaling pathway",
  "gene_symbol": "GPR101",
  "gene": "UniProtKB:Q96P66",
  "term_id": "GO:0071880",
  "gene_name": "Probable G-protein coupled receptor 101"
}